{
  "term_id": "GO:0005634",
  "gene_name": "Transcription elongation regulator 1",
  "gene": "UniProtKB:O14776",
  "term_label": "nucleus",
  "gene_symbol": "TCERG1"
}